{
  "gene": "UniProtKB:Q8IYM9",
  "term_label": "positive regulation of autophagy",
  "term_id": "GO:0010508",
  "gene_symbol": "TRIM22",
  "gene_name": "E3 ubiquitin-protein ligase TRIM22"
}